{
  "gene_symbol": "OPALIN",
  "gene": "UniProtKB:Q96PE5",
  "term_id": "GO:0044291",
  "gene_name": "Opalin",
  "term_label": "cell-cell contact zone"
}